{
  "term_label": "Unknown molecular function",
  "gene_name": "BolA-like protein 1",
  "gene_symbol": "BOLA1",
  "term_id": "UNKNOWN:0001",
  "gene": "UniProtKB:Q9Y3E2"
}